{
  "term_id": "GO:0005886",
  "gene_symbol": "MYMK",
  "term_label": "plasma membrane",
  "gene_name": "Protein myomaker",
  "gene": "UniProtKB:A6NI61"
}